glucosinolate metabolic process [GO:0019760] (biological process) Relationships: is a type of sulfur compound metabolic process [GO:0006790]; is a type of oxoacid metabolic process [GO:0043436]; is_a carbohydrate derivative metabolic process [GO:1901135] Subtypes: GO:0019761, glucosinolate catabolic process [GO:0019762], GO:0042343 Definition: The chemical reactions and pathways involving glucosinolates, substituted thioglucosides found in rapeseed products and related cruciferae. They are metabolized to a variety of toxic products which are most likely the cause of hepatocytic necrosis in animals and humans. Sources: GOC:curators Also known as: glucosinolate metabolism